{
  "term_label": "RNA polymerase II general transcription initiation factor activity",
  "gene": "UniProtKB:A0A1W2PPL8",
  "term_id": "GO:0016251",
  "gene_symbol": "TAF11L14",
  "gene_name": "TATA-box-binding protein-associated factor 11-like protein 14"
}